{
  "term_label": "phosphatidylinositol phosphate biosynthetic process",
  "term_id": "GO:0046854",
  "gene_name": "Phosphatidylinositol 5-phosphate 4-kinase type-2 gamma",
  "gene_symbol": "PIP4K2C",
  "gene": "UniProtKB:Q8TBX8"
}